plastid large ribosomal subunit [GO:0000311] (cellular component) Definition: The larger of the two subunits of a plastid ribosome. Two sites on the ribosomal large subunit are involved in translation: the aminoacyl site (A site) and peptidyl site (P site). Sources: GOC:mcc Relationships: is a type of organellar large ribosomal subunit [GO:0000315]; is part of plastid ribosome [GO:0009547] Subtypes: chloroplast large ribosomal subunit [GO:0022628]